{
  "gene": "UniProtKB:Q6ZMJ4",
  "term_id": "GO:0008284",
  "gene_symbol": "IL34",
  "gene_name": "Interleukin-34",
  "term_label": "positive regulation of cell population proliferation"
}